{
  "gene_symbol": "DNAH17",
  "gene": "UniProtKB:Q9UFH2",
  "term_id": "GO:0097729",
  "term_label": "9+2 motile cilium",
  "gene_name": "Dynein axonemal heavy chain 17"
}